{
  "gene_name": "COMM domain-containing protein 2",
  "term_label": "Unknown biological process",
  "term_id": "UNKNOWN:0002",
  "gene_symbol": "COMMD2",
  "gene": "UniProtKB:Q86X83"
}